{
  "term_id": "UNKNOWN:0003",
  "term_label": "Unknown cellular component",
  "gene_symbol": "FOLH1B",
  "gene": "UniProtKB:Q9HBA9",
  "gene_name": "Putative N-acetylated-alpha-linked acidic dipeptidase"
}